{
  "gene_symbol": "HNRNPA1",
  "gene_name": "Heterogeneous nuclear ribonucleoprotein A1",
  "gene": "UniProtKB:P09651",
  "term_label": "catalytic step 2 spliceosome",
  "term_id": "GO:0071013"
}